{
  "term_label": "insulin-like growth factor receptor signaling pathway",
  "gene": "UniProtKB:P08069",
  "term_id": "GO:0048009",
  "gene_symbol": "IGF1R",
  "gene_name": "Insulin-like growth factor 1 receptor"
}